{
  "gene_name": "Inositol monophosphatase 1",
  "term_id": "UNKNOWN:0003",
  "gene_symbol": "IMPA1",
  "term_label": "Unknown cellular component",
  "gene": "UniProtKB:P29218"
}